{
  "gene_name": "Protein tweety homolog 1",
  "gene_symbol": "TTYH1",
  "term_label": "plasma membrane",
  "gene": "UniProtKB:Q9H313",
  "term_id": "GO:0005886"
}